{
  "gene_symbol": "PSAP",
  "term_id": "UNKNOWN:0001",
  "term_label": "Unknown molecular function",
  "gene": "UniProtKB:P07602",
  "gene_name": "Prosaposin"
}